{
  "gene": "UniProtKB:Q8IVC4",
  "gene_symbol": "ZNF584",
  "term_id": "GO:0000981",
  "gene_name": "Zinc finger protein 584",
  "term_label": "DNA-binding transcription factor activity, RNA polymerase II-specific"
}